{
  "gene": "UniProtKB:P29966",
  "term_label": "actin filament organization",
  "gene_name": "Myristoylated alanine-rich C-kinase substrate",
  "gene_symbol": "MARCKS",
  "term_id": "GO:0007015"
}